{
  "term_label": "Unknown biological process",
  "gene": "UniProtKB:Q9BYR9",
  "term_id": "UNKNOWN:0002",
  "gene_symbol": "KRTAP2-4",
  "gene_name": "Keratin-associated protein 2-4"
}